{
  "gene_name": "Protein RIC-3",
  "term_id": "UNKNOWN:0001",
  "gene_symbol": "RIC3",
  "gene": "UniProtKB:Q7Z5B4",
  "term_label": "Unknown molecular function"
}